perisynaptic space [GO:0099544] (cellular component) Sources: GOC:dos Definition: The extracellular region immediately adjacent to to a synapse. Also known as: extrasynaptic space Relationships: is a type of extracellular region [GO:0005576]